negative regulation of miRNA processing [GO:1903799] (biological process) Also known as: down regulation of gene silencing by miRNA, production of miRNAs, down regulation of miRNA processing, down regulation of miRNA-mediated gene silencing, production of miRNAs, down regulation of microRNA-mediated gene silencing, production of microRNAs, down regulation of production of miRNAs involved in gene silencing by miRNA, down regulation of production of microRNAs involved in gene silencing by microRNA, down-regulation of gene silencing by miRNA, production of miRNAs, down-regulation of miRNA processing, down-regulation of miRNA-mediated gene silencing, production of miRNAs, down-regulation of microRNA-mediated gene silencing, production of microRNAs, down-regulation of production of miRNAs involved in gene silencing by miRNA, down-regulation of production of microRNAs involved in gene silencing by microRNA, downregulation of gene silencing by miRNA, production of miRNAs, downregulation of miRNA processing, downregulation of miRNA-mediated gene silencing, production of miRNAs, downregulation of microRNA-mediated gene silencing, production of microRNAs, downregulation of production of miRNAs involved in gene silencing by miRNA, downregulation of production of microRNAs involved in gene silencing by microRNA, negative regulation of gene silencing by miRNA, production of miRNAs, negative regulation of miRNA-mediated gene silencing, production of miRNAs, negative regulation of microRNA-mediated gene silencing, production of microRNAs, negative regulation of production of microRNAs involved in gene silencing by microRNA, inhibition of gene silencing by miRNA, production of miRNAs, inhibition of miRNA processing, inhibition of miRNA-mediated gene silencing, production of miRNAs, inhibition of microRNA-mediated gene silencing, production of microRNAs, inhibition of production of miRNAs involved in gene silencing by miRNA, inhibition of production of microRNAs involved in gene silencing by microRNA, negative regulation of miRNA maturation, down regulation of miRNA biogenesis, down regulation of microRNA biogenesis, down regulation of microRNA biosynthesis, down regulation of microRNA biosynthetic process, down regulation of microRNA metabolic process, down regulation of microRNA metabolism, down-regulation of miRNA biogenesis, down-regulation of microRNA biogenesis, down-regulation of microRNA biosynthesis, down-regulation of microRNA biosynthetic process, down-regulation of microRNA metabolic process, down-regulation of microRNA metabolism, downregulation of miRNA biogenesis, downregulation of microRNA biogenesis, downregulation of microRNA biosynthesis, downregulation of microRNA biosynthetic process, downregulation of microRNA metabolic process, downregulation of microRNA metabolism, inhibition of miRNA biogenesis, inhibition of microRNA biogenesis, inhibition of microRNA biosynthesis, inhibition of microRNA biosynthetic process, inhibition of microRNA metabolic process, inhibition of microRNA metabolism, negative regulation of miRNA biogenesis, negative regulation of microRNA biogenesis, negative regulation of microRNA biosynthesis, negative regulation of microRNA biosynthetic process, negative regulation of microRNA metabolic process, negative regulation of microRNA metabolism, negative regulation of production of miRNAs involved in gene silencing by miRNA Definition: Any process that stops, prevents or reduces the frequency, rate or extent of microRNA processing. Relationships: is_a negative regulation of gene expression [GO:0010629]; is a type of negative regulation of miRNA-mediated gene silencing [GO:0060965]; is a type of regulation of miRNA processing [GO:1903798]; RO_0002212 miRNA processing [GO:0035196] Subtypes: negative regulation of pre-miRNA processing [GO:2000632], negative regulation of primary miRNA processing [GO:2000635] References: PMID:22269326 Sources: GOC:BHF, GOC:BHF_miRNA, GOC:TermGenie, GOC:rph, GO_REF:0000058